regulation of activin secretion [GO:0032335] (biological process) Subtypes: negative regulation of activin secretion [GO:0032336], positive regulation of activin secretion [GO:0032337] Relationships: is a type of regulation of hormone secretion [GO:0046883]; regulates GO:0032333 Definition: Any process that modulates the frequency, rate or extent of the regulated release of activin from a cell. Sources: GOC:mah